{
  "gene_name": "Histone-lysine N-methyltransferase SETMAR",
  "term_label": "DNA topoisomerase binding",
  "term_id": "GO:0044547",
  "gene_symbol": "SETMAR",
  "gene": "UniProtKB:Q53H47"
}